{
  "term_id": "GO:0016020",
  "gene_symbol": "TAS2R10",
  "gene_name": "Taste receptor type 2 member 10",
  "gene": "UniProtKB:Q9NYW0",
  "term_label": "membrane"
}